{
  "gene": "UniProtKB:P09496",
  "term_id": "GO:0030125",
  "term_label": "clathrin vesicle coat",
  "gene_symbol": "CLTA",
  "gene_name": "Clathrin light chain A"
}